{
  "gene_name": "Neutrophil cytosol factor 4",
  "gene": "UniProtKB:Q15080",
  "gene_symbol": "NCF4",
  "term_label": "superoxide anion generation",
  "term_id": "GO:0042554"
}